clathrin-coated endocytic vesicle lumen [GO:0106176] (cellular component) Definition: The volume enclosed by the membrane of a clathrin-coated endocytic vesicle. Relationships: is_a endocytic vesicle lumen [GO:0071682]; is part of GO:0045334 References: PMID:2516741 Sources: GOC:pde